RNA exon ligation [GO:0000378] (biological process) Relationships: is a type of RNA metabolic process [GO:0016070]; is part of RNA splicing, via endonucleolytic cleavage and ligation [GO:0000394] Sources: GOC:krc, ISBN:0879695897 Definition: The RNA metabolic process that joins two exons, each of which has free ends that were generated by endonucleolytic cleavages, by a ligation reaction. Subtypes: tRNA exon ligation [GO:0000968] Note: Note that this is not a part of spliceosomal RNA splicing.